positive regulation of receptor localization to synapse [GO:1902685] (biological process) Also known as: positive regulation of receptor localisation to synapse, up regulation of receptor localisation to synapse, up regulation of receptor localization to synapse, up-regulation of receptor localisation to synapse, up-regulation of receptor localization to synapse, upregulation of receptor localisation to synapse, upregulation of receptor localization to synapse, activation of receptor localisation to synapse, activation of receptor localization to synapse Relationships: is a type of positive regulation of biological process [GO:0048518]; is a type of regulation of receptor localization to synapse [GO:1902683]; positively regulates receptor localization to synapse [GO:0097120] References: PMID:22252129 Sources: GOC:TermGenie, GOC:kmv, GO_REF:0000058 Definition: Any process that activates or increases the frequency, rate or extent of receptor localization to synapse.